cyclin-dependent protein kinase activity [GO:0097472] (molecular function) Relationships: is a type of protein kinase activity [GO:0004672]; is part of regulation of cell cycle [GO:0051726]; has part GO:0030332 Note: This reaction requires the binding of a regulatory cyclin subunit and full activity requires stimulatory phosphorylation by a CDK-activating kinase (CAK). Subtypes: GO:0004693 Regulation: regulated by cyclin-dependent protein kinase regulator activity [GO:0019914]; negatively regulated by negative regulation of cyclin-dependent protein kinase activity [GO:1904030]; positively regulated by positive regulation of cyclin-dependent protein kinase activity [GO:1904031] Sources: GOC:pr Definition: Cyclin-dependent catalysis of the phosphorylation of an amino acid residue in a protein, usually according to the reaction: a protein + ATP = a phosphoprotein + ADP.